{
  "gene_name": "Mediator of RNA polymerase II transcription subunit 23",
  "gene": "UniProtKB:Q9ULK4",
  "term_id": "GO:0006357",
  "gene_symbol": "MED23",
  "term_label": "regulation of transcription by RNA polymerase II"
}